mitochondrial DNA catabolic process [GO:0032043] (biological process) Relationships: is a type of DNA catabolic process [GO:0006308]; is a type of mitochondrial DNA metabolic process [GO:0032042] Also known as: mitochondrial DNA breakdown, mitochondrial DNA catabolism, mitochondrial DNA degradation, mtDNA breakdown, mtDNA catabolic process, mtDNA catabolism, mtDNA degradation Definition: The chemical reactions and pathways resulting in the breakdown of mitochondrial DNA. Sources: GOC:mah